{
  "gene_name": "Sulfotransferase 1E1",
  "term_label": "aryl sulfotransferase activity",
  "term_id": "GO:0004062",
  "gene": "UniProtKB:P49888",
  "gene_symbol": "SULT1E1"
}